{
  "gene": "UniProtKB:Q13069",
  "term_label": "Unknown biological process",
  "gene_symbol": "GAGE5",
  "term_id": "UNKNOWN:0002",
  "gene_name": "G antigen 5"
}